{
  "term_id": "GO:0043123",
  "gene": "UniProtKB:Q9HC29",
  "gene_symbol": "NOD2",
  "term_label": "positive regulation of canonical NF-kappaB signal transduction",
  "gene_name": "Nucleotide-binding oligomerization domain-containing protein 2"
}